embryo sac cellularization [GO:0009558] (biological process) Relationships: is a type of GO:0007349; is part of megagametogenesis [GO:0009561] Also known as: cellularization of the embryo sac, female gametophyte cellularization, megagametophyte cellularization Definition: The process in which the eight-nucleate single celled female gametophyte develops into the seven-celled female gametophyte. This mature structure contains two synergid cells and an egg cell at the micropylar end, and three antipodal cells at the other end. A binucleate endosperm mother cell is formed at the center. An example of this process is found in Arabidopsis thaliana. Sources: GOC:jid, GOC:mtg_plant, GOC:mtg_sensu, ISBN:047186840X